core TFIIH complex portion of holo TFIIH complex [GO:0000438] (cellular component) Relationships: is a type of transcription factor TFIIH core complex [GO:0000439]; is part of GO:0005675 Also known as: SSL2-core TFIIH complex portion of holo TFIIH complex Definition: The core TFIIH complex when it is part of the general transcription factor TFIIH. References: PMID:14500720, PMID:22308316, PMID:22572993, PMID:7813015 Sources: GOC:ew, GOC:krc